5S rRNA primary transcript binding [GO:0008098] (molecular function) Definition: Binding to an unprocessed 5S ribosomal RNA transcript. Relationships: is a type of 5S rRNA binding [GO:0008097] Sources: GOC:jl